{
  "gene_symbol": "CD300LF",
  "gene_name": "CMRF35-like molecule 1",
  "term_id": "GO:0002757",
  "gene": "UniProtKB:Q8TDQ1",
  "term_label": "immune response-activating signaling pathway"
}